{
  "term_id": "UNKNOWN:0001",
  "gene": "UniProtKB:Q9H3C7",
  "term_label": "Unknown molecular function",
  "gene_name": "Gametogenetin-binding protein 2",
  "gene_symbol": "GGNBP2"
}